{
  "gene_symbol": "RNF182",
  "term_label": "cytoplasm",
  "term_id": "GO:0005737",
  "gene": "UniProtKB:Q8N6D2",
  "gene_name": "E3 ubiquitin-protein ligase RNF182"
}